{
  "term_label": "Unknown biological process",
  "gene_symbol": "DPY19L1",
  "gene": "UniProtKB:Q2PZI1",
  "gene_name": "Probable C-mannosyltransferase DPY19L1",
  "term_id": "UNKNOWN:0002"
}